pyrroline-5-carboxylate reductase complex [GO:1902792] (cellular component) Definition: A protein complex which is capable of pyrroline-5-carboxylate reductase activity. Note: An example of this is PYCR1 in human (P32322) in PMID:2722838 (inferred from direct assay). Relationships: is a type of oxidoreductase complex [GO:1990204] References: PMID:2722838 Sources: GOC:TermGenie, GOC:bhm, GO_REF:0000088